{
  "gene_name": "Prefoldin subunit 1",
  "term_label": "unfolded protein binding",
  "term_id": "GO:0051082",
  "gene": "UniProtKB:O60925",
  "gene_symbol": "PFDN1"
}